{
  "term_label": "lactation",
  "gene_name": "Kappa-casein",
  "term_id": "GO:0007595",
  "gene": "UniProtKB:P07498",
  "gene_symbol": "CSN3"
}